{
  "term_id": "UNKNOWN:0002",
  "term_label": "Unknown biological process",
  "gene_symbol": "OR4M1",
  "gene_name": "Olfactory receptor 4M1",
  "gene": "UniProtKB:Q8NGD0"
}